rhombomere 1 formation [GO:0021652] (biological process) Definition: The process that gives rise to rhombomere 1. This process pertains to the initial formation of a structure from unspecified parts. Rhombomeres are transverse segments of the developing rhombencephalon. Rhombomeres are lineage restricted, express different genes from one another, and adopt different developmental fates. Rhombomeres are numbered in anterior to posterior order. Sources: GOC:cls, GOC:curators, GOC:dgh, GOC:dph, GOC:jid Relationships: is a type of GO:0021594; is part of rhombomere 1 morphogenesis [GO:0021651]